establishment of epithelial cell apical/basal polarity [GO:0045198] (biological process) Relationships: is a type of polarized epithelial cell differentiation [GO:0030859]; is a type of establishment of apical/basal cell polarity [GO:0035089]; is a type of GO:0045197; is_a establishment of epithelial cell polarity [GO:0090162] Definition: The specification and formation of the apicobasal polarity of an epithelial cell. Subtypes: establishment of myocardial progenitor cell apical/basal polarity [GO:0003316], establishment of epithelial cell apical/basal polarity involved in camera-type eye morphogenesis [GO:0003412] Sources: GOC:ascb_2009, GOC:bf, GOC:dph, GOC:tb